intracellularly ATP-gated calcium channel activity [GO:0140417] (molecular function) Definition: Enables the transmembrane transfer of a calcium ion from intracellular stores by a channel that opens when a ATP has been bound by the channel complex or one of its constituent parts. Relationships: is a type of intracellularly gated calcium channel activity [GO:0015278] Also known as: ATP-sensitive calcium-release channel activity References: PMID:22736763